cellular response to 3,3',5-triiodo-L-thyronine [GO:1905243] (biological process) Definition: Any process that results in a change in state or activity of a cell (in terms of movement, secretion, enzyme production, gene expression, etc.) as a result of a 3,3',5-triiodo-L-thyronine stimulus. References: PMID:21382270 Sources: GOC:TermGenie, GO_REF:0000071 Also known as: cellular response to Liothyronin, cellular response to Liothyronine, cellular response to Liothyroninum Relationships: is a type of cellular response to amino acid stimulus [GO:0071230]; is a type of cellular response to nitrogen compound [GO:1901699]; is_a cellular response to oxygen-containing compound [GO:1901701]; is a type of response to 3,3',5-triiodo-L-thyronine [GO:1905242]